type 1 fibroblast growth factor receptor binding [GO:0005105] (molecular function) Note: Note that breathless is the Drosophila gene encoding the type 1 fibroblast growth factor receptor (FGFR1). Also known as: FGFR1 binding, FGFR1 ligand, breathless binding, breathless ligand, type 1 fibroblast growth factor receptor ligand Definition: Binding to a type 1 fibroblast growth factor receptor (FGFR1). Sources: GOC:ceb, GOC:fb_curators Relationships: is a type of fibroblast growth factor receptor binding [GO:0005104]